{
  "gene_name": "Zinc finger protein 630",
  "gene_symbol": "ZNF630",
  "gene": "UniProtKB:Q2M218",
  "term_id": "GO:0000978",
  "term_label": "RNA polymerase II cis-regulatory region sequence-specific DNA binding"
}